{
  "gene": "UniProtKB:Q8TBZ6",
  "gene_name": "tRNA methyltransferase 10 homolog A",
  "gene_symbol": "TRMT10A",
  "term_label": "cytosol",
  "term_id": "GO:0005829"
}